{
  "gene_symbol": "IGLJ6",
  "gene": "UniProtKB:A0A0A0MT93",
  "term_label": "Unknown biological process",
  "gene_name": "Immunoglobulin lambda joining 6 (Fragment)",
  "term_id": "UNKNOWN:0002"
}